{
  "gene_name": "Arf-GAP with dual PH domain-containing protein 2",
  "gene_symbol": "ADAP2",
  "term_id": "GO:0005547",
  "term_label": "phosphatidylinositol-3,4,5-trisphosphate binding",
  "gene": "UniProtKB:Q9NPF8"
}